{
  "gene_name": "UBA-like domain-containing protein 2",
  "gene_symbol": "UBALD2",
  "gene": "UniProtKB:Q8IYN6",
  "term_label": "Unknown molecular function",
  "term_id": "UNKNOWN:0001"
}